negative regulation of B cell receptor signaling pathway [GO:0050859] (biological process) Sources: GOC:ai Definition: Any process that stops, prevents, or reduces the frequency, rate or extent of signaling pathways initiated by the cross-linking of an antigen receptor on a B cell. Also known as: down regulation of B cell receptor signaling pathway, down-regulation of B cell receptor signaling pathway, downregulation of B cell receptor signaling pathway, negative regulation of B cell receptor signalling pathway, negative regulation of B lymphocyte receptor signaling pathway, negative regulation of B lymphocyte receptor signalling pathway, negative regulation of B-cell receptor signaling pathway, negative regulation of B-cell receptor signalling pathway, negative regulation of B-lymphocyte receptor signaling pathway, negative regulation of B-lymphocyte receptor signalling pathway, inhibition of B cell receptor signaling pathway Relationships: is a type of regulation of B cell receptor signaling pathway [GO:0050855]; is a type of negative regulation of antigen receptor-mediated signaling pathway [GO:0050858]; negatively regulates B cell receptor signaling pathway [GO:0050853]